{
  "term_label": "Unknown molecular function",
  "term_id": "UNKNOWN:0001",
  "gene": "UniProtKB:P08F94",
  "gene_symbol": "PKHD1",
  "gene_name": "Fibrocystin"
}